deoxyguanosine salvage [GO:0006180] (BP) Definition: Any process that generates deoxyguanosine from derivatives of it, without de novo synthesis. Relationships: is a type of GO:0042452; is a type of purine deoxyribonucleoside salvage [GO:0043098] Sources: GOC:jl